{
  "term_label": "Rap protein signal transduction",
  "gene_name": "Ras-related protein Rap-1b-like protein",
  "term_id": "GO:0032486",
  "gene_symbol": "RAP1BL",
  "gene": "UniProtKB:A6NIZ1"
}